{
  "term_label": "cytoplasm",
  "gene_symbol": "CCNG1",
  "gene_name": "Cyclin-G1",
  "gene": "UniProtKB:P51959",
  "term_id": "GO:0005737"
}